{
  "term_id": "GO:0006879",
  "term_label": "intracellular iron ion homeostasis",
  "gene": "UniProtKB:O75027",
  "gene_name": "Iron-sulfur clusters transporter ABCB7, mitochondrial",
  "gene_symbol": "ABCB7"
}